{
  "gene_name": "Forkhead box protein N3",
  "term_label": "cis-regulatory region sequence-specific DNA binding",
  "gene": "UniProtKB:O00409",
  "term_id": "GO:0000987",
  "gene_symbol": "FOXN3"
}